{
  "gene_name": "Transmembrane protein 50B",
  "gene_symbol": "TMEM50B",
  "gene": "UniProtKB:P56557",
  "term_id": "GO:0032511",
  "term_label": "late endosome to vacuole transport via multivesicular body sorting pathway"
}